oxidoreductase activity, acting on other nitrogenous compounds as donors, iron-sulfur protein as acceptor [GO:0016664] (molecular function) Also known as: oxidoreductase activity, acting on other nitrogenous compounds as donors, iron-sulphur protein as acceptor Relationships: is a type of oxidoreductase activity, acting on other nitrogenous compounds as donors [GO:0016661] Subtypes: ferredoxin-nitrate reductase activity [GO:0047889], ferredoxin-nitrite reductase activity [GO:0048307] Definition: Catalysis of an oxidation-reduction (redox) reaction in which a nitrogenous group, excluding NH and NH2 groups, acts as a hydrogen or electron donor and reduces an iron-sulfur protein. Sources: EC:1.7.7.-